putrescine catabolic process [GO:0009447] (biological process) Definition: The chemical reactions and pathways resulting in the breakdown of putrescine, 1,4-diaminobutane; putrescine is the metabolic precursor of spermidine and spermine. Sources: GOC:ai Also known as: putrescine breakdown, putrescine catabolism, putrescine degradation Relationships: is a type of polyamine catabolic process [GO:0006598]; is a type of GO:0009445